positive regulation of postsynaptic density assembly [GO:0160036] (biological process) Relationships: is a type of regulation of postsynaptic density assembly [GO:0099151]; is a type of positive regulation of organelle assembly [GO:1902117]; is a type of positive regulation of postsynaptic density organization [GO:1905876]; RO_0002213 postsynaptic density assembly [GO:0097107] Definition: Any process that activates or increases the frequency, rate or extent of postsynaptic density assembly. References: PMID:17626212